{
  "gene": "UniProtKB:P78324",
  "gene_symbol": "SIRPA",
  "term_label": "Unknown molecular function",
  "term_id": "UNKNOWN:0001",
  "gene_name": "Tyrosine-protein phosphatase non-receptor type substrate 1"
}